negative regulation of T cell homeostatic proliferation [GO:0046014] (biological process) Sources: GOC:go_curators Relationships: is a type of negative regulation of T cell proliferation [GO:0042130]; is a type of regulation of T cell homeostatic proliferation [GO:0046013]; negatively regulates GO:0001777 Also known as: down regulation of T cell homeostatic proliferation, down-regulation of T cell homeostatic proliferation, downregulation of T cell homeostatic proliferation, negative regulation of T lymphocyte homeostatic proliferation, negative regulation of T-cell homeostatic proliferation, negative regulation of T-lymphocyte homeostatic proliferation, negative regulation of resting T cell proliferation, inhibition of T cell homeostatic proliferation Definition: Any process that stops, prevents or reduces the rate or extent of resting T cell proliferation.